transmitter-gated channel activity [GO:0022835] (molecular function) Definition: Enables the transmembrane transfer of a solute by a channel that opens when a specific neurotransmitter has been bound by the channel complex or one of its constituent parts. Sources: GOC:mtg_transport, ISBN:0815340729 Also known as: extracellular substance gated channel activity, neurotransmitter-gated channel activity Relationships: is a type of ligand-gated channel activity [GO:0022834]; is a type of neurotransmitter receptor activity [GO:0030594] Subtypes: GO:0022824